{
  "gene": "UniProtKB:Q8WXS5",
  "gene_symbol": "CACNG8",
  "term_label": "transmission of nerve impulse",
  "gene_name": "Voltage-dependent calcium channel gamma-8 subunit",
  "term_id": "GO:0019226"
}